response to thiabendazole [GO:0072712] (biological process) Relationships: is a type of response to nitrogen compound [GO:1901698] Sources: GOC:mah Definition: Any process that results in a change in state or activity of a cell or an organism (in terms of movement, secretion, enzyme production, gene expression, etc.) as a result of a thiabendazole stimulus. Also known as: response to TBZ Subtypes: cellular response to thiabendazole [GO:0072713]